{
  "gene": "UniProtKB:O00445",
  "gene_name": "Synaptotagmin-5",
  "gene_symbol": "SYT5",
  "term_label": "axon",
  "term_id": "GO:0030424"
}